methane biosynthetic process from dimethyl sulfide [GO:2001131] (biological process) Definition: The chemical reactions and pathways resulting in the formation of a methane from a dimethyl sulfide. Sources: GOC:mengo_curators Relationships: is a type of sulfur compound metabolic process [GO:0006790]; is_a methanogenesis [GO:0015948] Regulation: regulated by regulation of methane biosynthetic process from dimethyl sulfide [GO:1900342]; negatively regulated by negative regulation of methane biosynthetic process from dimethyl sulfide [GO:1900343]; positively regulated by positive regulation of methane biosynthetic process from dimethyl sulfide [GO:1900344]